regulation of vascular associated smooth muscle cell proliferation [GO:1904705] (biological process) Relationships: is a type of GO:0048660; RO_0002211 vascular associated smooth muscle cell proliferation [GO:1990874] Also known as: regulation of VSMC proliferation, regulation of vascular smooth muscle cell proliferation Subtypes: negative regulation of vascular associated smooth muscle cell proliferation [GO:1904706], positive regulation of vascular associated smooth muscle cell proliferation [GO:1904707] References: PMID:23246467 Sources: GOC:TermGenie, GO_REF:0000058 Definition: Any process that modulates the frequency, rate or extent of vascular smooth muscle cell proliferation.